proboscis morphogenesis, labial disc-derived [GO:0010782] (biological process) Definition: The process in which the anatomical structures of the proboscis that are derived from the labial disc are generated and organized. Sources: GOC:dph, GOC:tb Relationships: is a type of post-embryonic animal morphogenesis [GO:0009886]; is part of labial disc morphogenesis [GO:0007454]; is part of GO:0048734